heme transmembrane transport [GO:0035351] (biological process) Definition: The process in which heme, any compound of iron complexed in a porphyrin (tetrapyrrole) ring, is transported from one side of a membrane to the other by means of some agent such as a transporter or pore. Subtypes: heme export from vacuole to cytoplasm [GO:0140357], heme import across plasma membrane [GO:1904334] Note: Note that this term is not intended for use in annotating lateral movement within membranes. Sources: GOC:bf Relationships: is a type of heme transport [GO:0015886]; is a type of GO:0034755 Also known as: heme membrane transport